{
  "gene_name": "Thymocyte selection-associated high mobility group box protein TOX",
  "gene": "UniProtKB:O94900",
  "gene_symbol": "TOX",
  "term_label": "chromatin DNA binding",
  "term_id": "GO:0031490"
}